{
  "term_label": "Unknown biological process",
  "gene_name": "Proteasome assembly chaperone 3",
  "term_id": "UNKNOWN:0002",
  "gene_symbol": "PSMG3",
  "gene": "UniProtKB:Q9BT73"
}